positive regulation of synaptic vesicle priming [GO:0010808] (biological process) Relationships: is_a regulation of synaptic vesicle priming [GO:0010807]; is a type of GO:0031334; positively regulates synaptic vesicle priming [GO:0016082] References: PMID:15489511 Sources: GOC:dph, GOC:kmv, GOC:tb Definition: Any process that increases the frequency, rate or extent of synaptic vesicle priming. Synaptic vesicle priming is the formation of SNARE-containing complexes, bringing synaptic vesicle membrane and plasma membranes into close proximity and thereby facilitating membrane fusion.